keratan sulfate proteoglycan metabolic process [GO:0042339] (biological process) Subtypes: keratan sulfate proteoglycan biosynthetic process [GO:0018146], keratan sulfate proteoglycan catabolic process [GO:0042340] Definition: The chemical reactions and pathways involving keratan sulfate proteoglycans, which consist of a core protein linked to a keratan sulfate glycosaminoglycan. The keratan sulfate chain is composed of the repeating disaccharide unit beta-(1,4)-N-acetyl-D-glucosamine-beta-(1,3)-galactose, both of which can be sulfated. References: PMID:29340594 Relationships: is a type of proteoglycan metabolic process [GO:0006029] Also known as: keratan sulfate metabolism, keratan sulphate metabolic process, keratan sulphate metabolism